fructose catabolic process to hydroxyacetone phosphate and glyceraldehyde-3-phosphate [GO:0061624] (biological process) Definition: The chemical reactions and pathways resulting in the breakdown of fructose that results in the formation of dihydroxyacetone phosphate and glyceraldehyde-3-phosphate. Sources: GOC:dph, ISBN:0201090910 Relationships: is a type of fructose catabolic process [GO:0006001]; is a type of glyceraldehyde-3-phosphate metabolic process [GO:0019682]; has part GO:0004454; has part triokinase activity [GO:0050354]; has part fructose-1-phosphate aldolase activity [GO:0061609]